{
  "term_label": "RNA polymerase II transcription regulatory region sequence-specific DNA binding",
  "term_id": "GO:0000977",
  "gene": "UniProtKB:P0CI00",
  "gene_symbol": "ZNF705B",
  "gene_name": "Putative zinc finger protein 705B"
}